{
  "term_label": "external side of plasma membrane",
  "term_id": "GO:0009897",
  "gene_name": "Protein disulfide-isomerase",
  "gene": "UniProtKB:P07237",
  "gene_symbol": "P4HB"
}